extracellular space [GO:0005615] (CC) Relationships: is a type of cellular anatomical structure [GO:0110165]; is part of extracellular region [GO:0005576] Also known as: intercellular space Note: Note that for multicellular organisms, the extracellular space refers to everything outside a cell, but still within the organism (excluding the extracellular matrix). Gene products from a multi-cellular organism that are secreted from a cell into the interstitial fluid or blood can therefore be annotated to this term. Definition: That part of a multicellular organism outside the cells proper, usually taken to be outside the plasma membranes, and occupied by fluid. Sources: ISBN:0198547684